{
  "gene_name": "Dynamin-like 120 kDa protein, mitochondrial",
  "gene": "UniProtKB:O60313",
  "gene_symbol": "OPA1",
  "term_id": "GO:0008053",
  "term_label": "mitochondrial fusion"
}